{
  "gene_name": "Neutral amino acid transporter 9",
  "term_id": "GO:0015179",
  "gene": "UniProtKB:Q8NBW4",
  "term_label": "L-amino acid transmembrane transporter activity",
  "gene_symbol": "SLC38A9"
}